{
  "term_label": "plasma membrane",
  "gene_name": "Sodium_hydrogen exchanger 3",
  "term_id": "GO:0005886",
  "gene": "UniProtKB:P48764",
  "gene_symbol": "SLC9A3"
}